{
  "gene": "UniProtKB:Q02962",
  "term_id": "GO:0000981",
  "gene_symbol": "PAX2",
  "term_label": "DNA-binding transcription factor activity, RNA polymerase II-specific",
  "gene_name": "Paired box protein Pax-2"
}